positive regulation of vacuolar transport [GO:1903337] (biological process) Sources: GOC:TermGenie, GOC:vw, GO_REF:0000058 Also known as: up regulation of vacuolar transport, up-regulation of vacuolar transport, upregulation of vacuolar transport, activation of vacuolar transport Definition: Any process that activates or increases the frequency, rate or extent of vacuolar transport. Subtypes: positive regulation of protein targeting to vacuolar membrane [GO:1900485], positive regulation of late endosome to lysosome transport [GO:1902824], positive regulation of protein targeting to vacuole involved in autophagy [GO:1904053] Relationships: is a type of positive regulation of intracellular transport [GO:0032388]; is a type of regulation of vacuolar transport [GO:1903335]; positively regulates vacuolar transport [GO:0007034]